calcium ion homeostasis [GO:0055074] (biological process) Sources: GOC:ceb, GOC:jid, GOC:mah Definition: Any process involved in the maintenance of an internal steady state of calcium ions within an organism or cell. Subtypes: GO:0006874 Relationships: is a type of GO:0055080; is_a inorganic ion homeostasis [GO:0098771] Also known as: regulation of calcium ion concentration